positive regulation of mitotic spindle formation (spindle phase one) [GO:0110161] (BP) Relationships: is a type of positive regulation of mitotic spindle organization [GO:0110028]; is a type of regulation of mitotic spindle formation (spindle phase one) [GO:0110159]; is a type of GO:1905832; positively regulates mitotic spindle formation (spindle phase one) [GO:0061804] Sources: GOC:vw Definition: Any process that activates or increases the frequency, rate or extent of the cell cycle process in which the distance is lengthened between poles of the mitotic spindle during mitotic prophase (spindle phase one).